{
  "term_label": "chromatin binding",
  "gene": "UniProtKB:Q96RY5",
  "gene_name": "Protein cramped-like",
  "term_id": "GO:0003682",
  "gene_symbol": "CRAMP1"
}